synthetic cannabinoid binding [GO:1904483] (molecular function) Definition: Binding to synthetic cannabinoid. Relationships: is a type of binding [GO:0005488] References: PMID:10700562 Sources: GOC:TermGenie, GOC:mr, GO_REF:0000067